{
  "gene_symbol": "KBTBD3",
  "term_id": "GO:0043161",
  "gene": "UniProtKB:Q8NAB2",
  "gene_name": "Kelch repeat and BTB domain-containing protein 3",
  "term_label": "proteasome-mediated ubiquitin-dependent protein catabolic process"
}